glutathione transmembrane transporter activity [GO:0034634] (molecular function) Sources: GOC:mah Relationships: is a type of tripeptide transmembrane transporter activity [GO:0042937]; is a type of modified amino acid transmembrane transporter activity [GO:0072349]; is a type of sulfur compound transmembrane transporter activity [GO:1901682]; is part of GO:0034775 Definition: Enables the transfer of glutathione, the tripeptide glutamylcysteinylglycine, from one side of a membrane to the other.